positive regulation of cation channel activity [GO:2001259] (biological process) Subtypes: positive regulation of store-operated calcium channel activity [GO:1901341], positive regulation of voltage-gated calcium channel activity [GO:1901387], positive regulation of large conductance calcium-activated potassium channel activity [GO:1902608], GO:1903818, positive regulation of voltage-gated sodium channel activity [GO:1905152], GO:1905273 Sources: GOC:BHF Also known as: positive regulation of cation diffusion facilitator activity, positive regulation of nonselective cation channel activity Definition: Any process that activates or increases the frequency, rate or extent of cation channel activity. Relationships: is a type of GO:0032414; is a type of positive regulation of cation transmembrane transport [GO:1904064]; positively regulates monoatomic cation channel activity [GO:0005261]